{
  "gene_name": "GDP-fucose transporter 1",
  "term_label": "GDP-fucose import into Golgi lumen",
  "gene": "UniProtKB:Q96A29",
  "term_id": "GO:0036085",
  "gene_symbol": "SLC35C1"
}